{
  "term_id": "GO:0016791",
  "gene_name": "Phosphoethanolamine_phosphocholine phosphatase",
  "gene": "UniProtKB:Q8TCT1",
  "gene_symbol": "PHOSPHO1",
  "term_label": "phosphatase activity"
}